{
  "gene": "UniProtKB:Q9BSW7",
  "term_id": "GO:0016192",
  "gene_symbol": "SYT17",
  "gene_name": "Synaptotagmin-17",
  "term_label": "vesicle-mediated transport"
}